hydroxyglutamate decarboxylase activity [GO:0047990] (molecular function) Definition: Catalysis of the reaction: 3-hydroxy-L-glutamate + H+ = 4-amino-3-hydroxybutanoate + CO2. Sources: EC:4.1.1.16, RHEA:14073 Also known as: 3-hydroxy-L-glutamate 1-carboxy-lyase (4-amino-3-hydroxybutanoate-forming), 3-hydroxy-L-glutamate 1-carboxy-lyase activity Relationships: is_a carboxy-lyase activity [GO:0016831]